{
  "gene": "UniProtKB:Q8WUT9",
  "term_id": "UNKNOWN:0003",
  "term_label": "Unknown cellular component",
  "gene_symbol": "SLC25A43",
  "gene_name": "Solute carrier family 25 member 43"
}